{
  "term_id": "GO:0007188",
  "term_label": "adenylate cyclase-modulating G protein-coupled receptor signaling pathway",
  "gene": "UniProtKB:P11488",
  "gene_name": "Guanine nucleotide-binding protein G(t) subunit alpha-1",
  "gene_symbol": "GNAT1"
}